{
  "gene": "UniProtKB:A1L453",
  "term_id": "GO:0006508",
  "gene_symbol": "PRSS38",
  "term_label": "proteolysis",
  "gene_name": "Serine protease 38"
}